membrane-membrane adaptor activity [GO:0140177] (MF) Definition: The binding activity of a molecule that brings together two membranes, either via membrane lipid binding or by interacting with a membrane protein, to establish or maintain the localization of the protein, protein complex or organelle. Sources: GOC:curator Relationships: is a type of molecular adaptor activity [GO:0060090]